polygalacturonate 4-alpha-galacturonosyltransferase activity [GO:0047262] (molecular function) Definition: Catalysis of the reaction: UDP-D-galacturonate + 1,4-alpha-D-galacturonosyl(n) = 1,4-alpha-D-galacturonosyl(n+1) + UDP. Relationships: is a type of UDP-glycosyltransferase activity [GO:0008194]; is a type of hexosyltransferase activity [GO:0016758] Also known as: UDP galacturonate-polygalacturonate alpha-galacturonosyltransferase activity, UDP-D-galacturonate:1,4-alpha-poly-D-galacturonate 4-alpha-D-galacturonosyltransferase activity, uridine diphosphogalacturonate-polygalacturonate alpha-galacturonosyltransferase activity Sources: EC:2.4.1.43, MetaCyc:2.4.1.43-RXN